{
  "gene_symbol": "MEIKIN",
  "gene_name": "Meiosis-specific kinetochore protein",
  "gene": "UniProtKB:A0A087WXM9",
  "term_id": "UNKNOWN:0001",
  "term_label": "Unknown molecular function"
}